{
  "term_id": "GO:0008017",
  "gene_symbol": "CLASP1",
  "term_label": "microtubule binding",
  "gene_name": "CLIP-associating protein 1",
  "gene": "UniProtKB:Q7Z460"
}